{
  "gene_name": "Small nuclear ribonucleoprotein F",
  "term_label": "RNA binding",
  "gene": "UniProtKB:P62306",
  "term_id": "GO:0003723",
  "gene_symbol": "SNRPF"
}